pyrimidine-containing compound catabolic process [GO:0072529] (biological process) Sources: GOC:mah Subtypes: pyrimidine nucleobase catabolic process [GO:0006208], pyrimidine nucleotide catabolic process [GO:0006244], thiamine-containing compound catabolic process [GO:0042725], pyrimidine nucleoside catabolic process [GO:0046135] Relationships: is a type of GO:0009056; is a type of pyrimidine-containing compound metabolic process [GO:0072527] Definition: The chemical reactions and pathways resulting in the breakdown of a pyrimidine-containing compound, i.e. any compound that contains pyrimidine or a formal derivative thereof. Also known as: pyrimidine and derivative catabolic process, pyrimidine-containing compound breakdown, pyrimidine-containing compound catabolism, pyrimidine-containing compound degradation